collagen and cuticulin-based cuticle attachment to epithelium [GO:0040004] (biological process) Sources: GOC:ems, GOC:mtg_sensu Definition: Attaching of a collagen and cuticulin-based cuticle to the epithelium underlying it. An example of this process is found in Caenorhabditis elegans. Also known as: cuticular attachment to epithelium Relationships: is a type of molting cycle process [GO:0022404]; is part of molting cycle, collagen and cuticulin-based cuticle [GO:0018996]